MHC class II protein binding [GO:0042289] (molecular function) Definition: Binding to a major histocompatibility complex class II molecule; a set of molecules displayed on cell surfaces that are responsible for lymphocyte recognition and antigen presentation. Sources: GOC:jl Also known as: major histocompatibility complex class II binding, major histocompatibility complex class II ligand Note: Note that this term does not include binding to the antigen peptide bound to the MHC protein. Consider also annotating to the molecular function term 'peptide antigen binding ; GO:0042605' or one of its children. Relationships: is a type of MHC protein binding [GO:0042287] Subtypes: MHC class II protein binding, via lateral surface [GO:0042657], MHC class II protein binding, via antigen binding groove [GO:0042658]